symbiont-mediated activation of host inflammasome-mediated signal transduction [GO:0141079] (BP) Relationships: is a type of symbiont-mediated activation of host signal transduction pathway [GO:0052028] Also known as: perturbation of host inflammasome-mediated signal transduction Definition: A process in which a symbiont subverts an inflammasome-mediated signal transduction pathway in the host organism by initiating, promoting, or enhancing its activation. The host is defined as the larger of the organisms involved in a symbiotic interaction. References: PMID:25538194, PMID:28331908, PMID:30872531, PMID:34155776